negative regulation of protein kinase C signaling [GO:0090038] (biological process) Relationships: is a type of GO:0090036; is a type of negative regulation of intracellular signal transduction [GO:1902532]; negatively regulates protein kinase C signaling [GO:0070528] Also known as: negative regulation of protein kinase C signaling cascade, negative regulation of protein kinase C signalling cascade Sources: GOC:dph, GOC:tb Definition: Any process that decreases the frequency, rate, or extent of a series of reactions, mediated by the intracellular serine/threonine kinase protein kinase C, which occurs as a result of a single trigger reaction or compound.